{
  "gene": "UniProtKB:P0CB38",
  "gene_name": "Polyadenylate-binding protein 4-like",
  "term_id": "GO:0005634",
  "gene_symbol": "PABPC4L",
  "term_label": "nucleus"
}